{
  "gene_symbol": "TOMM5",
  "gene_name": "Mitochondrial import receptor subunit TOM5 homolog",
  "gene": "UniProtKB:Q8N4H5",
  "term_id": "UNKNOWN:0002",
  "term_label": "Unknown biological process"
}